{
  "gene_name": "T cell receptor alpha variable 12-3",
  "term_id": "UNKNOWN:0002",
  "gene": "UniProtKB:A0A0B4J271",
  "term_label": "Unknown biological process",
  "gene_symbol": "TRAV12-3"
}